positive regulation of vascular endothelial growth factor production [GO:0010575] (biological process) Definition: Any process that increases or activates the frequency, rate, or extent of production of vascular endothelial growth factor. Sources: GOC:BHF, GOC:rl Relationships: is a type of positive regulation of cytokine production [GO:0001819]; is a type of regulation of vascular endothelial growth factor production [GO:0010574]; positively regulates vascular endothelial growth factor production [GO:0010573]